histone H3K9me2/3 reader activity [GO:0062072] (molecular function) References: PMID:30110338 Note: Comment: Note that the residue position corresponds to the canonical human H3 histone (UniProtKB:P84243); this residue is conserved across all eukaryotes. Residue 1 is the first residue following removal of the initiating Methionine (Met). Note that each histone is encoded by multiple genes, and sequences may vary across different genes within an organism. Relationships: is a type of histone H3 reader activity [GO:0140006] Definition: A histone reader that recognizes a histone H3 trimethylated at lysine 9. In some organisms, there is only H3K9me2, not H3K9me3, but this modification is recognized by homologous readers. Also known as: H3K9me3 modified histone binding, histone H3K9me2 reader activity, histone H3K9me3 reader activity